{
  "gene_symbol": "RNF113A",
  "gene": "UniProtKB:O15541",
  "term_label": "U2-type spliceosomal complex",
  "gene_name": "E3 ubiquitin-protein ligase RNF113A",
  "term_id": "GO:0005684"
}